{
  "gene_name": "Transcription initiation factor TFIID subunit 5",
  "term_id": "GO:0016251",
  "gene_symbol": "TAF5",
  "gene": "UniProtKB:Q15542",
  "term_label": "RNA polymerase II general transcription initiation factor activity"
}